{
  "term_label": "DNA-binding transcription factor activity, RNA polymerase II-specific",
  "gene_name": "Zinc finger protein 709",
  "gene": "UniProtKB:Q8N972",
  "gene_symbol": "ZNF709",
  "term_id": "GO:0000981"
}